{
  "gene": "UniProtKB:P0C2W7",
  "term_label": "Unknown molecular function",
  "gene_symbol": "CT47B1",
  "term_id": "UNKNOWN:0001",
  "gene_name": "Cancer_testis antigen family 47 member B1"
}